{
  "gene_symbol": "ZFP30",
  "gene": "UniProtKB:Q9Y2G7",
  "gene_name": "Zinc finger protein 30 homolog",
  "term_label": "DNA-binding transcription factor activity, RNA polymerase II-specific",
  "term_id": "GO:0000981"
}